{
  "gene_symbol": "AGER",
  "term_id": "GO:0038023",
  "term_label": "signaling receptor activity",
  "gene_name": "Advanced glycosylation end product-specific receptor",
  "gene": "UniProtKB:Q15109"
}